response to interleukin-2 [GO:0070669] (biological process) Sources: GOC:mah Definition: Any process that results in a change in state or activity of a cell or an organism (in terms of movement, secretion, enzyme production, gene expression, etc.) as a result of an interleukin-2 stimulus. Also known as: response to IL-2 Subtypes: cellular response to interleukin-2 [GO:0071352] Relationships: is a type of response to cytokine [GO:0034097]